central B cell selection [GO:0002340] (biological process) Sources: GOC:jal Subtypes: central B cell positive selection [GO:0002348], central B cell negative selection [GO:0002354] Also known as: central B lymphocyte selection, central B-cell selection, central B-lymphocyte selection Definition: Any B cell selection process that occurs in the bone marrow. Relationships: is a type of B cell selection [GO:0002339]